{
  "gene_symbol": "PDILT",
  "gene": "UniProtKB:Q8N807",
  "gene_name": "Protein disulfide-isomerase-like protein of the testis",
  "term_label": "endoplasmic reticulum",
  "term_id": "GO:0005783"
}